{
  "term_id": "GO:0007186",
  "gene_symbol": "GPR17",
  "gene": "UniProtKB:Q13304",
  "gene_name": "Uracil nucleotide_cysteinyl leukotriene receptor",
  "term_label": "G protein-coupled receptor signaling pathway"
}